{
  "gene_symbol": "MIR22HG",
  "gene": "UniProtKB:Q0VDD5",
  "term_id": "UNKNOWN:0001",
  "term_label": "Unknown molecular function",
  "gene_name": "Putative uncharacterized protein encoded by MIR22HG"
}